negative regulation of wax biosynthetic process [GO:1904277] (biological process) Definition: Any process that stops, prevents or reduces the frequency, rate or extent of wax biosynthetic process. References: PMID:24692420 Sources: GOC:TermGenie, GO_REF:0000058 Also known as: down regulation of wax anabolism, down regulation of wax biosynthesis, down regulation of wax biosynthetic process, down regulation of wax formation, down regulation of wax synthesis, down-regulation of wax anabolism, down-regulation of wax biosynthesis, down-regulation of wax biosynthetic process, down-regulation of wax formation, down-regulation of wax synthesis, downregulation of wax anabolism, downregulation of wax biosynthesis, downregulation of wax biosynthetic process, downregulation of wax formation, downregulation of wax synthesis, negative regulation of wax anabolism, negative regulation of wax biosynthesis, negative regulation of wax formation, negative regulation of wax synthesis, inhibition of wax anabolism, inhibition of wax biosynthesis, inhibition of wax biosynthetic process, inhibition of wax formation, inhibition of wax synthesis Relationships: is a type of negative regulation of lipid biosynthetic process [GO:0051055]; is a type of regulation of wax biosynthetic process [GO:1904276]; negatively regulates GO:0010025